triglyceride transport [GO:0034197] (BP) Definition: The directed movement of triglyceride into, out of or within a cell, or between cells, by means of some agent such as a transporter or pore. Triglycerides are important components of plant oils, animal fats and animal plasma lipoproteins. Regulation: regulated by regulation of triglyceride transport [GO:1905883]; negatively regulated by negative regulation of triglyceride transport [GO:1905884]; positively regulated by positive regulation of triglyceride transport [GO:1905885] Also known as: triacylglycerol transport Relationships: is a type of acylglycerol transport [GO:0034196] Sources: GOC:BHF, GOC:rl